{
  "term_label": "autophagosome assembly",
  "term_id": "GO:0000045",
  "gene_name": "Tumor protein p53-inducible nuclear protein 2",
  "gene_symbol": "TP53INP2",
  "gene": "UniProtKB:Q8IXH6"
}